plant-type cell wall cellulose catabolic process [GO:0044348] (biological process) Sources: GOC:mengo_curators Relationships: is a type of cell wall polysaccharide catabolic process [GO:0044347]; is a type of plant-type cell wall cellulose metabolic process [GO:0052541] Also known as: plant-type cell wall polysaccharide breakdown Regulation: regulated by regulation of plant-type cell wall cellulose catabolic process [GO:2000939]; negatively regulated by negative regulation of plant-type cell wall cellulose catabolic process [GO:2000940]; positively regulated by positive regulation of plant-type cell wall cellulose catabolic process [GO:2000941] Definition: The chemical reactions and pathways resulting in the breakdown of cellulose, a linear beta1-4 glucan of molecular mass 50-400 kDa with the pyranose units in the -4C1 conformation, which forms part of the cell wall.